ATPase-coupled hydroxyectoine transmembrane transporter activity [GO:0033288] (molecular function) Also known as: hydroxyectoine transmembrane transporter activity, ATP-dependent hydroxyectoine transmembrane transporter activity, hydroxyectoine-transporting ATPase activity Definition: Enables the transfer of a solute or solutes from one side of a membrane to the other according to the reaction: ATP + H2O + hydroxyectoine(out/in) = ADP + phosphate + hydroxyectoine(in/out). Relationships: is a type of quaternary ammonium group transmembrane transporter activity [GO:0015651]; is a type of alcohol transmembrane transporter activity [GO:0015665]; is a type of ATPase-coupled monocarboxylic acid transmembrane transporter activity [GO:0033285]; is part of hydroxyectoine transmembrane transport [GO:0033308] Sources: GOC:mlg